{
  "gene_symbol": "DEFB110",
  "gene": "UniProtKB:Q30KQ9",
  "term_id": "GO:0005615",
  "gene_name": "Beta-defensin 110",
  "term_label": "extracellular space"
}